{
  "gene": "UniProtKB:P09630",
  "term_label": "nucleus",
  "gene_name": "Homeobox protein Hox-C6",
  "gene_symbol": "HOXC6",
  "term_id": "GO:0005634"
}